{
  "term_id": "GO:0000398",
  "gene_symbol": "PRPF4",
  "gene": "UniProtKB:O43172",
  "term_label": "mRNA splicing, via spliceosome",
  "gene_name": "U4_U6 small nuclear ribonucleoprotein Prp4"
}